AP-5 adaptor complex [GO:0044599] (CC) Relationships: is a type of AP-type membrane coat adaptor complex [GO:0030119] References: PMID:22022230 Definition: An AP-type membrane coat adaptor complex that in humans consists of beta5, zeta, mu5 and sigma5 subunits and is found associated with membranes in the endosomes; it is not clear whether AP-5 forms clathrin coats in vivo. Also known as: adaptor protein-5 adaptor complex